positive regulation of aorta morphogenesis [GO:1903849] (biological process) Definition: Any process that activates or increases the frequency, rate or extent of aorta morphogenesis. Relationships: is a type of regulation of aorta morphogenesis [GO:1903847]; is a type of positive regulation of artery morphogenesis [GO:1905653]; positively regulates GO:0035909 Also known as: up regulation of aorta morphogenesis, up-regulation of aorta morphogenesis, upregulation of aorta morphogenesis, activation of aorta morphogenesis References: PMID:22269326 Sources: GOC:BHF, GOC:BHF_miRNA, GOC:TermGenie, GOC:rph, GO_REF:0000058